{
  "gene_symbol": "MYRF",
  "term_id": "GO:0005789",
  "gene_name": "Myelin regulatory factor",
  "gene": "UniProtKB:Q9Y2G1",
  "term_label": "endoplasmic reticulum membrane"
}